{
  "term_id": "GO:0015810",
  "gene_name": "Mitochondrial glutamate carrier 2",
  "term_label": "aspartate transmembrane transport",
  "gene": "UniProtKB:Q9H1K4",
  "gene_symbol": "SLC25A18"
}